pteridine-containing compound biosynthetic process [GO:0042559] (BP) Relationships: is_a biosynthetic process [GO:0009058]; is a type of pteridine-containing compound metabolic process [GO:0042558] Definition: The chemical reactions and pathways resulting in the formation of any compound containing pteridine (pyrazino(2,3-dipyrimidine)), e.g. pteroic acid, xanthopterin and folic acid. Subtypes: pteridine biosynthetic process [GO:0006728], tetrahydrobiopterin biosynthetic process [GO:0006729], GO:0009396, tatiopterin biosynthetic process [GO:1900870], methanopterin-containing compound biosynthetic process [GO:2001116] Also known as: pteridine and derivative biosynthesis, pteridine and derivative biosynthetic process, pteridine-containing compound anabolism, pteridine-containing compound biosynthesis, pteridine-containing compound formation, pteridine-containing compound synthesis, pterin biosynthesis, pterin biosynthetic process Sources: GOC:jl, ISBN:0198506732